cuticular extracellular matrix [GO:0060102] (cellular component) Definition: A collagen and cuticulin-based noncellular, multilayered structure that is synthesized by an underlying ectodermal (hypodermal) cell layer. The cuticle serves essential functions in body morphology, locomotion, and environmental protection. An example of this component is found in Caenorhabditis elegans. References: PMID:12619137 Sources: GOC:dph, GOC:kmv, ISSN:15518507 Also known as: collagen and cuticulin-based cuticle extracellular matrix, cuticular ECM, collagen and cuticulin-based exoskeleton extracellular matrix Relationships: is a type of specialized extracellular matrix [GO:0140047]